positive regulation of neutrophil chemotaxis [GO:0090023] (biological process) Sources: GOC:dph, GOC:tb Definition: Any process that increases the frequency, rate, or extent of neutrophil chemotaxis. Neutrophil chemotaxis is the directed movement of a neutrophil cell, the most numerous polymorphonuclear leukocyte found in the blood, in response to an external stimulus, usually an infection or wounding. Relationships: is a type of positive regulation of granulocyte chemotaxis [GO:0071624]; is a type of regulation of neutrophil chemotaxis [GO:0090022]; is a type of positive regulation of neutrophil migration [GO:1902624]; positively regulates neutrophil chemotaxis [GO:0030593]